protein nucleotidylation [GO:0018175] (biological process) Relationships: is a type of protein modification process [GO:0036211] Subtypes: protein adenylylation [GO:0018117], protein uridylylation [GO:0018177], protein guanylylation [GO:0018260] Sources: GOC:ai Also known as: protein amino acid nucleotidylation Definition: The addition of a nucleotide to a protein amino acid.